{
  "term_label": "Unknown cellular component",
  "gene": "UniProtKB:Q96SE0",
  "term_id": "UNKNOWN:0003",
  "gene_symbol": "ABHD1",
  "gene_name": "Protein ABHD1"
}